negative regulation of kinase activity [GO:0033673] (biological process) Definition: Any process that stops, prevents, or reduces the frequency, rate or extent of kinase activity, the catalysis of the transfer of a phosphate group, usually from ATP, to a substrate molecule. Sources: GOC:mah Also known as: down regulation of kinase activity, down-regulation of kinase activity, downregulation of kinase activity, inhibition of kinase activity, kinase inhibitor Relationships: is a type of GO:0042326; is a type of GO:0043086; is a type of regulation of kinase activity [GO:0043549]; negatively regulates kinase activity [GO:0016301] Subtypes: negative regulation of protein kinase activity [GO:0006469], negative regulation of glucokinase activity [GO:0033132]